{
  "gene": "UniProtKB:O00429",
  "term_label": "mitochondrion",
  "term_id": "GO:0005739",
  "gene_name": "Dynamin-1-like protein",
  "gene_symbol": "DNM1L"
}